{
  "gene_symbol": "IRF9",
  "gene": "UniProtKB:Q00978",
  "term_label": "immune system process",
  "gene_name": "Interferon regulatory factor 9",
  "term_id": "GO:0002376"
}